{
  "gene_symbol": "H1-3",
  "gene_name": "Histone H1.3",
  "gene": "UniProtKB:P16402",
  "term_id": "GO:0005634",
  "term_label": "nucleus"
}